{
  "gene_symbol": "HNF1A",
  "term_id": "GO:0000981",
  "gene": "UniProtKB:P20823",
  "gene_name": "Hepatocyte nuclear factor 1-alpha",
  "term_label": "DNA-binding transcription factor activity, RNA polymerase II-specific"
}